{
  "gene": "UniProtKB:A0A2R8Y4M2",
  "gene_name": "Uncharacterized protein",
  "term_id": "UNKNOWN:0002",
  "term_label": "Unknown biological process",
  "gene_symbol": "A0A2R8Y4M2"
}